{
  "term_label": "mitochondrial outer membrane translocase complex",
  "gene_symbol": "TOMM20L",
  "gene": "UniProtKB:Q6UXN7",
  "term_id": "GO:0005742",
  "gene_name": "TOMM20-like protein 1"
}